{
  "gene": "UniProtKB:P78423",
  "term_id": "GO:0006954",
  "gene_name": "Fractalkine",
  "gene_symbol": "CX3CL1",
  "term_label": "inflammatory response"
}